{
  "term_label": "N-acylsphingosine galactosyltransferase activity",
  "term_id": "GO:0003851",
  "gene_symbol": "UGT8",
  "gene": "UniProtKB:Q16880",
  "gene_name": "2-hydroxyacylsphingosine 1-beta-galactosyltransferase"
}